{
  "gene_symbol": "NINJ1",
  "gene": "UniProtKB:Q92982",
  "term_label": "pyroptotic cell death",
  "term_id": "GO:0141201",
  "gene_name": "Ninjurin-1"
}